{
  "term_id": "GO:0046870",
  "term_label": "cadmium ion binding",
  "gene": "UniProtKB:P49281",
  "gene_symbol": "SLC11A2",
  "gene_name": "Natural resistance-associated macrophage protein 2"
}